budding cell bud growth [GO:0007117] (biological process) Relationships: is a type of growth [GO:0040007]; is part of cell budding [GO:0007114] Definition: The process in which the bud portion of a cell that reproduces by budding irreversibly increases in size over time by accretion and biosynthetic production of matter similar to that already present. Also known as: bud growth Sources: GOC:go_curators Subtypes: budding cell apical bud growth [GO:0007118], GO:0007119